{
  "gene": "UniProtKB:Q9BXN6",
  "gene_symbol": "SPANXD",
  "gene_name": "Sperm protein associated with the nucleus on the X chromosome D",
  "term_id": "UNKNOWN:0002",
  "term_label": "Unknown biological process"
}